granulosa cell fate commitment [GO:0060015] (biological process) Sources: GOC:dph Definition: The cell fate commitment of precursor cells that will become granulosa cells. Relationships: is a type of epithelial cell fate commitment [GO:0072148]; is part of GO:0060014